{
  "gene_name": "Putative ADP-ribosylation factor-like protein 5C",
  "term_label": "trans-Golgi network",
  "term_id": "GO:0005802",
  "gene_symbol": "ARL5C",
  "gene": "UniProtKB:A6NH57"
}